{
  "gene_symbol": "FAS",
  "term_id": "GO:0097049",
  "term_label": "motor neuron apoptotic process",
  "gene": "UniProtKB:P25445",
  "gene_name": "Tumor necrosis factor receptor superfamily member 6"
}